{
  "term_id": "GO:0050869",
  "term_label": "negative regulation of B cell activation",
  "gene": "UniProtKB:Q8NDB2",
  "gene_name": "B-cell scaffold protein with ankyrin repeats",
  "gene_symbol": "BANK1"
}